{
  "term_id": "GO:0005085",
  "gene": "UniProtKB:Q9BZ29",
  "gene_name": "Dedicator of cytokinesis protein 9",
  "term_label": "guanyl-nucleotide exchange factor activity",
  "gene_symbol": "DOCK9"
}